{
  "gene_symbol": "ULBP2",
  "term_id": "GO:0046703",
  "gene": "UniProtKB:Q9BZM5",
  "term_label": "natural killer cell lectin-like receptor binding",
  "gene_name": "UL16-binding protein 2"
}